{
  "term_id": "GO:0003714",
  "gene_name": "B-cell lymphoma 3 protein",
  "gene": "UniProtKB:P20749",
  "term_label": "transcription corepressor activity",
  "gene_symbol": "BCL3"
}